phenylalanine 2-monooxygenase activity [GO:0050172] (molecular function) Sources: EC:1.13.12.9, RHEA:10712 Relationships: is a type of oxidoreductase activity, acting on single donors with incorporation of molecular oxygen, incorporation of one atom of oxygen (internal monooxygenases or internal mixed function oxidases) [GO:0016703] Definition: Catalysis of the reaction: L-phenylalanine + O2 = 2-phenylacetamide + CO2 + H2O. Also known as: L-phenylalanine oxidase (deaminating and decarboxylating), L-phenylalanine:oxygen 2-oxidoreductase (decarboxylating), l-phenylalanine oxidase (deaminating and decarboxylating) activity, phenylalanine (deaminating, decarboxylating) oxidase activity, phenylalanine (deaminating, decarboxylating)oxidase activity